{
  "gene_symbol": "OR5B12",
  "gene": "UniProtKB:Q96R08",
  "term_label": "odorant binding",
  "gene_name": "Olfactory receptor 5B12",
  "term_id": "GO:0005549"
}